{
  "gene_name": "Iron-sulfur protein NUBPL",
  "gene_symbol": "NUBPL",
  "term_id": "GO:0051539",
  "gene": "UniProtKB:Q8TB37",
  "term_label": "4 iron, 4 sulfur cluster binding"
}